{
  "term_label": "positive regulation of cell population proliferation",
  "gene_symbol": "PDGFC",
  "gene": "UniProtKB:Q9NRA1",
  "gene_name": "Platelet-derived growth factor C",
  "term_id": "GO:0008284"
}